{
  "gene": "UniProtKB:Q9P0V8",
  "term_label": "signaling receptor activity",
  "gene_symbol": "SLAMF8",
  "term_id": "GO:0038023",
  "gene_name": "SLAM family member 8"
}